cyanelle membrane [GO:0033113] (cellular component) Relationships: is a type of GO:0042170; is part of cyanelle envelope [GO:0033112] Subtypes: cyanelle inner membrane [GO:0036012], cyanelle outer membrane [GO:0036013] Sources: GOC:ecd Definition: Either of the lipid bilayers that surround a cyanelle and form the cyanelle envelope.